{
  "gene": "UniProtKB:P00568",
  "term_id": "UNKNOWN:0002",
  "gene_name": "Adenylate kinase isoenzyme 1",
  "gene_symbol": "AK1",
  "term_label": "Unknown biological process"
}